{
  "gene_symbol": "SCUBE3",
  "term_label": "Unknown molecular function",
  "gene_name": "Signal peptide, CUB and EGF-like domain-containing protein 3",
  "term_id": "UNKNOWN:0001",
  "gene": "UniProtKB:Q8IX30"
}